{
  "term_id": "GO:0006357",
  "term_label": "regulation of transcription by RNA polymerase II",
  "gene_symbol": "TADA2B",
  "gene": "UniProtKB:Q86TJ2",
  "gene_name": "Transcriptional adapter 2-beta"
}